nuclear androgen receptor binding [GO:0050681] (molecular function) Sources: GOC:ai Also known as: androgen receptor binding, AR binding Relationships: is a type of GO:0016922 Definition: Binding to a nuclear androgen receptor.